{
  "gene": "UniProtKB:P98164",
  "gene_name": "Low-density lipoprotein receptor-related protein 2",
  "term_id": "GO:0042562",
  "gene_symbol": "LRP2",
  "term_label": "hormone binding"
}